{
  "term_label": "GDP-D-glucose phosphorylase activity",
  "gene_name": "GDP-D-glucose phosphorylase 1",
  "gene": "UniProtKB:Q6ZNW5",
  "term_id": "GO:0080048",
  "gene_symbol": "GDPGP1"
}